{
  "gene_symbol": "OR2A25",
  "gene_name": "Olfactory receptor 2A25",
  "gene": "UniProtKB:A4D2G3",
  "term_label": "detection of chemical stimulus involved in sensory perception of smell",
  "term_id": "GO:0050911"
}